{
  "gene": "UniProtKB:Q9NQL2",
  "gene_name": "Ras-related GTP-binding protein D",
  "gene_symbol": "RRAGD",
  "term_label": "negative regulation of autophagy",
  "term_id": "GO:0010507"
}